negative regulation of nitric oxide mediated signal transduction [GO:0010751] (biological process) Definition: Any process that decreases the rate, frequency or extent of nitric oxide mediated signal transduction. Nitric oxide mediated signal transduction is The series of molecular signals mediated by the detection of nitric oxide (NO). Relationships: is a type of regulation of nitric oxide mediated signal transduction [GO:0010749]; is a type of negative regulation of intracellular signal transduction [GO:1902532]; negatively regulates GO:0007263 Subtypes: negative regulation of nitric oxide-cGMP mediated signal transduction [GO:0141151] Sources: GOC:BHF, GOC:dph, GOC:tb Also known as: negative regulation of nitric oxide-mediated signal transduction